condensed mesenchymal cell proliferation [GO:0072137] (biological process) Relationships: is a type of GO:0010463 Sources: GOC:mtg_kidney_jan10 Definition: The multiplication or reproduction of cells, resulting in the expansion of a condensed mesenchymal cell population. A condensed mesenchymal cell population is a population of adherent mesenchymal cells.